{
  "gene_name": "Myotubularin",
  "term_id": "GO:0052629",
  "gene": "UniProtKB:Q13496",
  "term_label": "phosphatidylinositol-3,5-bisphosphate 3-phosphatase activity",
  "gene_symbol": "MTM1"
}